{
  "term_label": "cysteine-type deubiquitinase activity",
  "gene_name": "Josephin-2",
  "term_id": "GO:0004843",
  "gene_symbol": "JOSD2",
  "gene": "UniProtKB:Q8TAC2"
}